{
  "gene_symbol": "ZNF586",
  "gene_name": "Zinc finger protein 586",
  "gene": "UniProtKB:Q9NXT0",
  "term_id": "GO:0000981",
  "term_label": "DNA-binding transcription factor activity, RNA polymerase II-specific"
}